cholesterol 26-hydroxylase activity [GO:0031073] (molecular function) Definition: Catalysis of the reaction: cholesterol + H+ NADPH + O2 = 26-hydroxycholesterol + H2O + NADP+. Relationships: is_a GO:0008395; is a type of GO:0016716 References: PMID:950499 Sources: RHEA:43836